positive regulation of antibacterial peptide biosynthetic process [GO:0006963] (biological process) Definition: Any process that activates or increases the frequency, rate, or extent of antibacterial peptide biosynthesis. References: PMID:10973475 Sources: GOC:mah Also known as: antibacterial peptide induction, antibacterial polypeptide induction, up regulation of antibacterial peptide biosynthetic process, up-regulation of antibacterial peptide biosynthetic process, upregulation of antibacterial peptide biosynthetic process, activation of antibacterial peptide biosynthetic process, stimulation of antibacterial peptide biosynthetic process Relationships: is a type of positive regulation of antibacterial peptide production [GO:0002803]; is a type of GO:0002807; is a type of regulation of antibacterial peptide biosynthetic process [GO:0002808]; positively regulates antibacterial peptide biosynthetic process [GO:0002780] Subtypes: GO:0006964, positive regulation of biosynthetic process of antibacterial peptides active against Gram-positive bacteria [GO:0006965]